pigment biosynthetic process [GO:0046148] (biological process) Definition: The chemical reactions and pathways resulting in the formation of a pigment, any general or particular coloring matter in living organisms, e.g. melanin. Sources: ISBN:0198506732 Also known as: pigment anabolism, pigment biosynthesis, pigment formation, pigment synthesis Relationships: is a type of pigment metabolic process [GO:0042440] Subtypes: eye pigment biosynthetic process [GO:0006726], pteridine biosynthetic process [GO:0006728], heme biosynthetic process [GO:0006783], ocellus pigment biosynthetic process [GO:0008055], anthocyanin-containing compound biosynthetic process [GO:0009718], chlorophyll biosynthetic process [GO:0015995], carotenoid biosynthetic process [GO:0016117], melanin biosynthetic process [GO:0042438], GO:0043477, phytochrome chromophore biosynthetic process [GO:0048543], aurone biosynthetic process [GO:0051551], GO:0051553, GO:0051559